linear primary-alkylsulfatase activity [GO:0018741] (molecular function) Relationships: is a type of sulfuric ester hydrolase activity [GO:0008484] Also known as: alkyl sulfatase activity Definition: Catalysis of the reaction: a primary linear alkyl sulfate ester + H2O = a primary alcohol + H+ + sulfate. Sources: RHEA:67908